{
  "term_id": "UNKNOWN:0002",
  "gene_symbol": "MSANTD4",
  "gene": "UniProtKB:Q8NCY6",
  "gene_name": "Myb_SANT-like DNA-binding domain-containing protein 4",
  "term_label": "Unknown biological process"
}